plasmacytoid dendritic cell differentiation [GO:0002273] (biological process) Definition: The process in which a relatively unspecialized hemopoietic precursor cell acquires the specialized features of a plasmacytoid dendritic cell. References: PMID:15990333, PMID:16174108 Sources: GOC:add Relationships: is a type of plasmacytoid dendritic cell activation [GO:0002270]; is a type of dendritic cell differentiation [GO:0097028] Subtypes: plasmacytoid dendritic cell differentiation involved in immune response [GO:0002272]